intramembranous ossification [GO:0001957] (biological process) Definition: Direct ossification that occurs within mesenchyme or an accumulation of relatively unspecialized cells. Note: An instance of intramembranous ossification may also be classified as metaplastic; the former classifies based on tissue type location, and the latter based on mechanism/cell division. Relationships: is a type of direct ossification [GO:0036072] Also known as: dermal ossification, intramembranous bone ossification Subtypes: GO:0036073 Sources: ISBN:0878932437